neuromuscular junction of myotube [GO:0098523] (cellular component) Relationships: is a type of GO:0031594 Definition: A neuromuscular junction in which the target muscle cell is a myotube. Subtypes: GO:0098522, neuromuscular junction of somatic muscle myotube [GO:0098524] Note: In vertebrates, the term 'neuromuscular junction' is limited to synapses targeting the myotubes of skeletal muscle (AKA skeletal muscle fibers). Neuromuscular junctions targeting other muscle cell types exist in invertebrates such as the mononucleate somatic muscles of nematodes. Sources: GOC:dos